{
  "gene": "UniProtKB:Q6ZVX9",
  "term_id": "UNKNOWN:0003",
  "term_label": "Unknown cellular component",
  "gene_name": "Membrane progestin receptor epsilon",
  "gene_symbol": "PAQR9"
}